{
  "term_label": "Unknown cellular component",
  "term_id": "UNKNOWN:0003",
  "gene_name": "Protein LSM14 homolog B",
  "gene_symbol": "LSM14B",
  "gene": "UniProtKB:Q9BX40"
}